{
  "gene": "UniProtKB:Q8N271",
  "term_id": "GO:0016324",
  "gene_symbol": "PROM2",
  "term_label": "apical plasma membrane",
  "gene_name": "Prominin-2"
}